{
  "gene": "UniProtKB:Q9NT99",
  "gene_symbol": "LRRC4B",
  "term_id": "GO:0099151",
  "gene_name": "Leucine-rich repeat-containing protein 4B",
  "term_label": "regulation of postsynaptic density assembly"
}